{
  "term_id": "UNKNOWN:0001",
  "gene_symbol": "LAMA4",
  "term_label": "Unknown molecular function",
  "gene_name": "Laminin subunit alpha-4",
  "gene": "UniProtKB:Q16363"
}